{
  "term_label": "Golgi apparatus",
  "term_id": "GO:0005794",
  "gene_symbol": "NDFIP2",
  "gene": "UniProtKB:Q9NV92",
  "gene_name": "NEDD4 family-interacting protein 2"
}